negative regulation of ribonucleoprotein complex localization [GO:2000198] (BP) Relationships: is a type of negative regulation of cellular process [GO:0048523]; is a type of regulation of ribonucleoprotein complex localization [GO:2000197]; negatively regulates ribonucleoprotein complex localization [GO:0071166] Sources: GOC:mah Subtypes: negative regulation of ribosomal subunit export from nucleus [GO:2000201], negative regulation of tRNA export from nucleus [GO:2000239] Definition: Any process that stops, prevents, or reduces the frequency, rate or extent of ribonucleoprotein complex localization. Also known as: negative regulation of RNP localization, negative regulation of cellular ribonucleoprotein complex localization, negative regulation of establishment and maintenance of ribonucleoprotein complex localization, negative regulation of ribonucleoprotein complex localisation